ectodermal placode morphogenesis [GO:0071697] (biological process) Definition: The process in which the anatomical structures of an ectodermal placode are generated and organized. An ectodermal placode is a thickening of the ectoderm that is the primordium of many structures derived from the ectoderm. Subtypes: olfactory placode morphogenesis [GO:0071699] Relationships: is a type of anatomical structure morphogenesis [GO:0009653]; is part of ectodermal placode development [GO:0071696] Sources: GOC:mah